peptidyl-cysteine S-nitrosylase activity [GO:0035605] (molecular function) Also known as: S-nitrosylase activity, protein nitrosylase activity Relationships: is_a transferase activity, transferring nitrogenous groups [GO:0016769]; is a type of catalytic activity, acting on a protein [GO:0140096] Note: This term should not be used to annotate the nitrosylating action of nitric oxide synthase (NOS) if the nitroso group is synthesized directly on the substrate. References: PMID:20972425, PMID:20972426 Sources: GOC:sp Definition: Catalysis of the transfer of a nitric oxide (NO) group to a sulphur atom within a cysteine residue of a protein.